{
  "gene": "UniProtKB:Q9Y261",
  "gene_symbol": "FOXA2",
  "term_id": "GO:0009653",
  "gene_name": "Hepatocyte nuclear factor 3-beta",
  "term_label": "anatomical structure morphogenesis"
}